{
  "gene": "UniProtKB:O43365",
  "term_label": "anterior/posterior pattern specification",
  "term_id": "GO:0009952",
  "gene_name": "Homeobox protein Hox-A3",
  "gene_symbol": "HOXA3"
}